{
  "gene_name": "Transmembrane protein 191B",
  "term_id": "UNKNOWN:0002",
  "gene_symbol": "TMEM191B",
  "gene": "UniProtKB:P0C7N4",
  "term_label": "Unknown biological process"
}